{
  "gene_symbol": "MPND",
  "gene": "UniProtKB:Q8N594",
  "term_label": "polyubiquitin modification-dependent protein binding",
  "gene_name": "MPN domain-containing protein",
  "term_id": "GO:0031593"
}